{
  "gene": "UniProtKB:O00515",
  "term_label": "Unknown cellular component",
  "gene_symbol": "LAD1",
  "gene_name": "Ladinin-1",
  "term_id": "UNKNOWN:0003"
}